{
  "gene_symbol": "HTR1A",
  "term_id": "GO:0051378",
  "term_label": "serotonin binding",
  "gene_name": "5-hydroxytryptamine receptor 1A",
  "gene": "UniProtKB:P08908"
}